{
  "term_label": "postsynaptic density",
  "gene_symbol": "PICK1",
  "gene": "UniProtKB:Q9NRD5",
  "term_id": "GO:0014069",
  "gene_name": "PRKCA-binding protein"
}